kolavenyl diphosphate synthase activity [GO:0106242] (MF) Relationships: is a type of GO:0016872 Definition: Catalysis of the reaction: all-trans-geranylgeranyl diphosphate = (+)-kolavenyl diphosphate. References: PMID:29315936 Sources: GOC:eab, RHEA:54676